{
  "term_label": "DNA-binding transcription factor activity, RNA polymerase II-specific",
  "term_id": "GO:0000981",
  "gene_name": "LIM homeobox transcription factor 1-alpha",
  "gene_symbol": "LMX1A",
  "gene": "UniProtKB:Q8TE12"
}